SREBP signaling pathway [GO:0032933] (biological process) Relationships: is a type of ER-nucleus signaling pathway [GO:0006984]; is a type of cellular response to sterol depletion [GO:0071501] Definition: The series of molecular signals from the endoplasmic reticulum to the nucleus generated as a consequence of decreased levels of one or more sterols (and in some yeast, changes in oxygen levels) and which proceeds through activation of a sterol response element binding transcription factor (SREBP) to result in up-regulation of target gene transcription. References: PMID:12923525, PMID:22017871 Sources: GOC:bf, GOC:mah, GOC:signaling, GOC:vw Regulation: regulated by regulation of SREBP signaling pathway [GO:2000638]; negatively regulated by negative regulation of SREBP signaling pathway [GO:2000639]; positively regulated by positive regulation of SREBP signaling pathway [GO:2000640] Also known as: sterol regulatory element binding protein target gene transcriptional activation, ER to nucleus sterol response pathway, ER-nuclear sterol response pathway, SREBP signalling, SREBP target gene transcriptional activation, SREBP-mediated signalling pathway, endoplasmic reticulum to nucleus sterol response pathway, endoplasmic reticulum-nuclear sterol response pathway, positive regulation of sterol regulatory element binding protein target gene transcription, positive regulation of sterol regulatory element binding protein target gene transcription involved in sterol depletion response, sterol depletion response, SREBP target gene transcriptional activation, sterol response element binding protein signaling pathway, up regulation of sterol regulatory element binding protein target gene transcription, up-regulation of sterol regulatory element binding protein target gene transcription, upregulation of sterol regulatory element binding protein target gene transcription, activation of sterol regulatory element binding protein target gene transcription, positive regulation of transcription via sterol regulatory element binding, positive regulation of transcription via sterol regulatory element binding involved in ER-nuclear sterol response pathway, stimulation of sterol regulatory element binding protein target gene transcription, SREBP-mediated signaling pathway